ilicicolin H biosynthetic process [GO:0140781] (biological process) References: PMID:30905148, PMID:31216742, PMID:34947016 Also known as: ilicicolin H anabolism, ilicicolin H biosynthesis, ilicicolin H formation, ilicicolin H synthesis Definition: The chemical reactions and pathways resulting in the formation of ilicicolin H, a 4-hydroxy-2-pyridone alkaloid that has potent and broad antifungal activities by inhibiting the mitochondrial respiration chain. Relationships: is a type of GO:0009821; is a type of polyketide biosynthetic process [GO:0030639]; is a type of GO:0042181; is a type of mycotoxin biosynthetic process [GO:0043386]; is a type of phenol-containing compound biosynthetic process [GO:0046189]; is a type of GO:0072525